{
  "gene_name": "Microtubule-associated proteins 1A_1B light chain 3 beta 2",
  "term_label": "cellular response to nitrogen starvation",
  "gene": "UniProtKB:A6NCE7",
  "gene_symbol": "MAP1LC3B2",
  "term_id": "GO:0006995"
}